{
  "gene_name": "Protein FAM3D",
  "gene": "UniProtKB:Q96BQ1",
  "gene_symbol": "FAM3D",
  "term_label": "cytokine activity",
  "term_id": "GO:0005125"
}